ionotropic bitter taste receptor activity [GO:0170022] (molecular function) Definition: Enables the transmembrane transfer of an ion by a channel that opens when a specific bitter compound has been bound by the channel complex or one of its constituent parts. Relationships: is a type of ionotropic taste receptor activity [GO:0170021] References: PMID:21262465